insemination [GO:0007320] (biological process) Relationships: is a type of multi-organism reproductive process [GO:0044703]; is a type of GO:0044706; is a type of GO:0048609; is part of copulation [GO:0007620] Sources: ISBN:0582227089 Definition: The introduction of semen or sperm into the genital tract of a female.